{
  "gene_name": "Harmonin",
  "term_id": "GO:0005886",
  "gene": "UniProtKB:Q9Y6N9",
  "term_label": "plasma membrane",
  "gene_symbol": "USH1C"
}